cellular extravasation [GO:0045123] (biological process) Relationships: is a type of leukocyte migration [GO:0050900] Also known as: immune cell cellular extravasation, leucocyte cellular extravasation, leukocyte cellular extravasation, transendothelial leukocyte migration Sources: GOC:jl Subtypes: monocyte extravasation [GO:0035696], neutrophil extravasation [GO:0072672], GO:0072682, T cell extravasation [GO:0072683] Definition: The migration of a leukocyte from the blood vessels into the surrounding tissue. Regulation: regulated by regulation of cellular extravasation [GO:0002691]; negatively regulated by negative regulation of cellular extravasation [GO:0002692]; positively regulated by positive regulation of cellular extravasation [GO:0002693]